{
  "term_id": "GO:0043047",
  "term_label": "single-stranded telomeric DNA binding",
  "gene": "UniProtKB:Q92878",
  "gene_name": "DNA repair protein RAD50",
  "gene_symbol": "RAD50"
}